{
  "gene_name": "DNA repair-scaffolding protein",
  "gene": "UniProtKB:Q14159",
  "gene_symbol": "SPIDR",
  "term_label": "nuclear chromosome",
  "term_id": "GO:0000228"
}